{
  "gene": "UniProtKB:P55263",
  "term_id": "GO:0006144",
  "gene_name": "Adenosine kinase",
  "term_label": "purine nucleobase metabolic process",
  "gene_symbol": "ADK"
}